{
  "gene_name": "Hepatocyte growth factor-like protein",
  "term_label": "receptor tyrosine kinase binding",
  "gene_symbol": "MST1",
  "gene": "UniProtKB:P26927",
  "term_id": "GO:0030971"
}